negative regulation of cap-independent translational initiation [GO:1903678] (biological process) Also known as: down regulation of cap-independent translational initiation, down-regulation of cap-independent translational initiation, downregulation of cap-independent translational initiation, inhibition of cap-independent translational initiation Relationships: is a type of regulation of cap-independent translational initiation [GO:1903677]; is a type of negative regulation of cytoplasmic translational initiation [GO:1904689]; negatively regulates cap-independent translational initiation [GO:0002190] Definition: Any process that stops, prevents or reduces the frequency, rate or extent of cap-independent translational initiation. Sources: GOC:PARL, GOC:TermGenie, GOC:bf, GO_REF:0000058